{
  "term_label": "structural constituent of ribosome",
  "gene": "UniProtKB:Q13084",
  "gene_name": "Large ribosomal subunit protein bL28m",
  "gene_symbol": "MRPL28",
  "term_id": "GO:0003735"
}